{
  "gene_name": "Solute carrier organic anion transporter family member 4C1",
  "gene": "UniProtKB:Q6ZQN7",
  "gene_symbol": "SLCO4C1",
  "term_label": "sodium-independent organic anion transport",
  "term_id": "GO:0043252"
}